{
  "term_id": "UNKNOWN:0001",
  "gene": "UniProtKB:Q7L099",
  "gene_symbol": "RUFY3",
  "term_label": "Unknown molecular function",
  "gene_name": "Protein RUFY3"
}